{
  "gene_symbol": "MARCHF5",
  "gene_name": "E3 ubiquitin-protein ligase MARCHF5",
  "term_label": "protein polyubiquitination",
  "term_id": "GO:0000209",
  "gene": "UniProtKB:Q9NX47"
}